{
  "gene_symbol": "GABRB1",
  "gene": "UniProtKB:P18505",
  "term_label": "GABA-A receptor complex",
  "term_id": "GO:1902711",
  "gene_name": "Gamma-aminobutyric acid receptor subunit beta-1"
}